{
  "gene_symbol": "GNB4",
  "term_label": "G protein-coupled receptor signaling pathway",
  "term_id": "GO:0007186",
  "gene": "UniProtKB:Q9HAV0",
  "gene_name": "Guanine nucleotide-binding protein subunit beta-4"
}